neuron projection regeneration [GO:0031102] (biological process) Relationships: is a type of GO:0031099; is a type of GO:0031175; is a type of cellular response to stress [GO:0033554] Regulation: RO_0002211 by regulation of neuron projection regeneration [GO:0070570]; negatively regulated by negative regulation of neuron projection regeneration [GO:0070571]; positively regulated by positive regulation of neuron projection regeneration [GO:0070572] Sources: GOC:dgh, GOC:dph, GOC:tb Definition: The regrowth of neuronal processes such as axons or dendrites in response to their loss or damage. Subtypes: axon regeneration [GO:0031103], GO:0031104 Also known as: neurite regeneration